{
  "term_id": "GO:0045332",
  "gene_symbol": "ATP10B",
  "gene": "UniProtKB:O94823",
  "term_label": "phospholipid translocation",
  "gene_name": "Phospholipid-transporting ATPase VB"
}